{
  "term_label": "Unknown biological process",
  "gene_symbol": "SERINC3",
  "term_id": "UNKNOWN:0002",
  "gene_name": "Serine incorporator 3",
  "gene": "UniProtKB:Q13530"
}